catechin binding [GO:0097246] (MF) Definition: Binding to a catechin, a polyphenolic antioxidant plant metabolite with a flavonoid or flavan-3-ol structure. Relationships: is_a flavanol binding [GO:0097245] Sources: GOC:sl